daunorubicin transport [GO:0043215] (biological process) Relationships: is a type of organic cation transport [GO:0015695]; is a type of nitrogen compound transport [GO:0071705]; is a type of glycoside transport [GO:1901656] Sources: GOC:jl, GOC:mlg Definition: The directed movement of daunorubicin, an anthracycline antibiotic produced by Streptomyces coeruleorubidus or S. peucetius and used as an antineoplastic into, out of or within a cell, or between cells, by means of some agent such as a transporter or pore.